{
  "gene_symbol": "MANEA",
  "gene_name": "Glycoprotein endo-alpha-1,2-mannosidase",
  "gene": "UniProtKB:Q5SRI9",
  "term_label": "alpha-mannosidase activity",
  "term_id": "GO:0004559"
}